{
  "gene_symbol": "FAM20B",
  "gene": "UniProtKB:O75063",
  "gene_name": "Glycosaminoglycan xylosylkinase",
  "term_id": "GO:0030166",
  "term_label": "proteoglycan biosynthetic process"
}